chenodeoxycholic acid binding [GO:1902122] (molecular function) Definition: Binding to chenodeoxycholic acid. References: PMID:10334992 Sources: GOC:TermGenie, GOC:bf Also known as: CDCA binding Relationships: is a type of steroid binding [GO:0005496]; is a type of bile acid binding [GO:0032052]